{
  "gene_symbol": "FBLIM1",
  "term_id": "GO:0098609",
  "gene_name": "Filamin-binding LIM protein 1",
  "term_label": "cell-cell adhesion",
  "gene": "UniProtKB:Q8WUP2"
}